purine nucleoside monophosphate biosynthetic process [GO:0009127] (biological process) Definition: The chemical reactions and pathways resulting in the formation of purine nucleoside monophosphate, a compound consisting of a purine base linked to a ribose or deoxyribose sugar esterified with phosphate on the sugar. Subtypes: purine ribonucleoside monophosphate biosynthetic process [GO:0009168], purine deoxyribonucleoside monophosphate biosynthetic process [GO:0009171] Also known as: purine nucleoside monophosphate anabolism, purine nucleoside monophosphate biosynthesis, purine nucleoside monophosphate formation, purine nucleoside monophosphate synthesis Relationships: is a type of nucleoside monophosphate biosynthetic process [GO:0009124]; is a type of purine nucleoside monophosphate metabolic process [GO:0009126] Sources: GOC:go_curators, ISBN:0198506732